{
  "gene_symbol": "ELK1",
  "term_id": "GO:0000981",
  "term_label": "DNA-binding transcription factor activity, RNA polymerase II-specific",
  "gene_name": "ETS domain-containing protein Elk-1",
  "gene": "UniProtKB:P19419"
}